{
  "gene_name": "Disintegrin and metalloproteinase domain-containing protein 32",
  "term_id": "GO:0007339",
  "term_label": "binding of sperm to zona pellucida",
  "gene": "UniProtKB:Q8TC27",
  "gene_symbol": "ADAM32"
}